{
  "gene_name": "Microfibrillar-associated protein 5",
  "gene": "UniProtKB:Q13361",
  "term_label": "Unknown molecular function",
  "gene_symbol": "MFAP5",
  "term_id": "UNKNOWN:0001"
}